{
  "gene_name": "U3 small nucleolar RNA-associated protein 14 homolog A",
  "gene": "UniProtKB:Q9BVJ6",
  "term_label": "Unknown molecular function",
  "gene_symbol": "UTP14A",
  "term_id": "UNKNOWN:0001"
}